{
  "gene_symbol": "CSKMT",
  "term_id": "GO:0016279",
  "term_label": "protein-lysine N-methyltransferase activity",
  "gene": "UniProtKB:A8MUP2",
  "gene_name": "Citrate synthase-lysine N-methyltransferase CSKMT, mitochondrial"
}